fumarate reductase (NADH) activity [GO:0016156] (molecular function) Definition: Catalysis of the reaction: NAD+ + succinate = fumarate + H+ + NADH. Relationships: is a type of succinate dehydrogenase activity [GO:0000104]; is a type of oxidoreductase activity, acting on the CH-CH group of donors, NAD or NADP as acceptor [GO:0016628] Also known as: NADH-dependent fumarate reductase activity Sources: RHEA:18281